cis-p-coumarate glucosyltransferase activity [GO:0050644] (molecular function) Relationships: is a type of UDP-glucosyltransferase activity [GO:0035251] Definition: Catalysis of the reaction: cis-4-coumarate + UDP-D-glucose = 4'-O-beta-D-glucosyl-cis-4-coumarate + H+ + UDP. Sources: EC:2.4.1.209, RHEA:13129 Also known as: UDP-glucose:cis-p-coumarate beta-D-glucosyltransferase activity